{
  "gene_symbol": "GLG1",
  "term_label": "fibroblast growth factor binding",
  "gene_name": "Golgi apparatus protein 1",
  "term_id": "GO:0017134",
  "gene": "UniProtKB:Q92896"
}